{
  "gene_symbol": "TLR8",
  "term_id": "GO:0032755",
  "gene": "UniProtKB:Q9NR97",
  "term_label": "positive regulation of interleukin-6 production",
  "gene_name": "Toll-like receptor 8"
}